basal labyrinth [GO:0033774] (cellular component) Definition: A region in the lower half of some cells formed from extensive infoldings of the basal plasma membrane; includes cytoplasm adjacent to the infolded membrane. Relationships: is a type of GO:0110165; is part of GO:0045178 References: PMID:11640882 Sources: GOC:mah, GOC:sart